establishment of planar polarity involved in mesonephric nephron morphogenesis [GO:0061238] (biological process) Relationships: is_a establishment of planar polarity involved in nephron morphogenesis [GO:0072046]; is part of mesonephric nephron morphogenesis [GO:0061228] Also known as: establishment of planar cell polarity involved in mesonephric nephron morphogenesis Definition: Coordinated organization of groups of cells in the plane of an epithelium that contributes to the shaping of a nephron in the mesonephros. Sources: GOC:mtg_kidney_jan10